{
  "term_label": "Unknown cellular component",
  "gene_name": "APRG1 tumor suppressor candidate",
  "term_id": "UNKNOWN:0003",
  "gene_symbol": "APRG1",
  "gene": "UniProtKB:Q8IVJ8"
}